2-oxo-hept-3-ene-1,7-dioate hydratase activity [GO:0018817] (molecular function) Definition: Catalysis of the reaction: cis-2-oxohept-3-ene-1,7-dioate + H2O = 2,4-dihydroxy-hept-trans-2-ene-1,7-dioate. Relationships: is a type of GO:0016836 Sources: UM-BBD_reactionID:r0369 Also known as: 2-oxo-hepta-3-ene-1,7-dioate hydratase activity, 2-oxo-hepta-3-ene-1,7-dioic acid hydratase activity, HpaH